{
  "term_label": "Unknown cellular component",
  "term_id": "UNKNOWN:0003",
  "gene": "UniProtKB:P52788",
  "gene_name": "Spermine synthase",
  "gene_symbol": "SMS"
}